sodium:dicarboxylate symporter activity [GO:0017153] (molecular function) Subtypes: GO:0015361, high-affinity sodium:dicarboxylate symporter activity [GO:0015362], malate:sodium symporter activity [GO:0043882], sodium:malonate symporter activity [GO:0044668] Also known as: sodium:dicarboxylate cotransporter activity Sources: GOC:ai Definition: Enables the transfer of a solute or solutes from one side of a membrane to the other according to the reaction: dicarboxylate(out) + Na+(out) = dicarboxylate(in) + Na+(in). Relationships: is a type of GO:0005310; is a type of GO:0005343